{
  "gene_name": "Ras-related protein Rab-27A",
  "gene_symbol": "RAB27A",
  "term_label": "exocytosis",
  "term_id": "GO:0006887",
  "gene": "UniProtKB:P51159"
}